plasmacytoid dendritic cell activation involved in immune response [GO:0002271] (biological process) References: PMID:15990333, PMID:16174109 Sources: GOC:add Relationships: is a type of plasmacytoid dendritic cell activation [GO:0002270]; is_a GO:0002366 Subtypes: plasmacytoid dendritic cell differentiation involved in immune response [GO:0002272] Definition: A change in the morphology or behavior of a plasmacytoid dendritic cell resulting from exposure to an activating factor such as a cellular or soluble ligand, leading to the initiation or perpetuation of an immune response. Also known as: plasmacytoid dendritic cell activation during immune response